negative regulation of fear response [GO:1903366] (biological process) References: PMID:8677262 Sources: GOC:TermGenie, GOC:mr, GO_REF:0000058 Also known as: down regulation of fear response, down regulation of physiological fear response, down-regulation of fear response, down-regulation of physiological fear response, downregulation of fear response, downregulation of physiological fear response, negative regulation of physiological fear response, inhibition of fear response, inhibition of physiological fear response Relationships: is a type of negative regulation of response to stimulus [GO:0048585]; is a type of negative regulation of multicellular organismal process [GO:0051241]; is a type of GO:1903365; negatively regulates fear response [GO:0042596] Subtypes: GO:2000986 Definition: Any process that stops, prevents or reduces the frequency, rate or extent of fear response.